{
  "gene_name": "Prion-like protein doppel",
  "term_label": "cellular response to copper ion",
  "term_id": "GO:0071280",
  "gene": "UniProtKB:Q9UKY0",
  "gene_symbol": "PRND"
}